{
  "term_id": "GO:0006623",
  "term_label": "protein targeting to vacuole",
  "gene": "UniProtKB:Q9H9H4",
  "gene_symbol": "VPS37B",
  "gene_name": "Vacuolar protein sorting-associated protein 37B"
}